{
  "term_label": "Unknown biological process",
  "term_id": "UNKNOWN:0002",
  "gene": "UniProtKB:Q53RE8",
  "gene_name": "Ankyrin repeat domain-containing protein 39",
  "gene_symbol": "ANKRD39"
}